{
  "term_id": "GO:0004493",
  "term_label": "methylmalonyl-CoA epimerase activity",
  "gene": "UniProtKB:Q96PE7",
  "gene_name": "Methylmalonyl-CoA epimerase, mitochondrial",
  "gene_symbol": "MCEE"
}